{
  "gene": "UniProtKB:Q8NET5",
  "term_label": "transmembrane signaling receptor activity",
  "gene_symbol": "NFAM1",
  "term_id": "GO:0004888",
  "gene_name": "NFAT activation molecule 1"
}